{
  "gene": "UniProtKB:A0A494C1R9",
  "term_id": "GO:0003682",
  "term_label": "chromatin binding",
  "gene_symbol": "TSPY9",
  "gene_name": "Testis-specific Y-encoded protein 9"
}